{
  "gene": "UniProtKB:Q8N1L1",
  "term_id": "UNKNOWN:0003",
  "term_label": "Unknown cellular component",
  "gene_name": "Putative uncharacterized protein encoded by LINC00528",
  "gene_symbol": "LINC00528"
}